{
  "term_label": "sodium-dependent phosphate transport",
  "term_id": "GO:0044341",
  "gene_name": "Sodium-dependent phosphate transport protein 2C",
  "gene_symbol": "SLC34A3",
  "gene": "UniProtKB:Q8N130"
}